RNA polyadenylation at postsynapse [GO:0140235] (biological process) References: PMID:22727665 Note: Note that this term was created for the SynGO project, and will be obsoleted when the SynGO annotations are made in Noctua. Definition: A polyadenylation event (the enzymatic addition of a sequence of adenylyl residues at the 3' end of an RNA molecule) that takes place at a postsynapse. Relationships: is a type of RNA processing [GO:0006396]